{
  "term_label": "Unknown molecular function",
  "gene_symbol": "TMEM242",
  "gene": "UniProtKB:Q9NWH2",
  "gene_name": "Transmembrane protein 242",
  "term_id": "UNKNOWN:0001"
}